calcitonin family receptor signaling pathway [GO:0097646] (biological process) Subtypes: amylin receptor signaling pathway [GO:0097647], calcitonin gene-related peptide receptor signaling pathway [GO:1990408], adrenomedullin receptor signaling pathway [GO:1990410] Relationships: is a type of G protein-coupled receptor signaling pathway [GO:0007186] References: PMID:10871296, PMID:12037140, PMID:18687416 Sources: GOC:bhm Also known as: calcitonin family receptor signalling pathway Definition: A G protein-coupled receptor signaling pathway initiated by an extracellular member of the calcitonin family (e.g. adrenomedullin, adrenomedullin 2 (intermedin), amylin, calcitonin and calcitonin gene-related peptides (CGRPs)) binding to its receptor on the surface of a target cell, and ending with the regulation of a downstream cellular process.